carnitinamidase activity [GO:0047773] (molecular function) Also known as: L-carnitinamidase activity, L-carnitinamide amidohydrolase activity, L-carnitine amidase activity, carnitine amidase activity Relationships: is a type of hydrolase activity, acting on carbon-nitrogen (but not peptide) bonds, in linear amides [GO:0016811] Definition: Catalysis of the reaction: (R)-carnitinamide + H2O = (R)-carnitine + NH4. Sources: EC:3.5.1.73, RHEA:17537